{
  "gene_name": "Tectonic-2",
  "gene_symbol": "TCTN2",
  "term_id": "UNKNOWN:0001",
  "term_label": "Unknown molecular function",
  "gene": "UniProtKB:Q96GX1"
}